P-TEFb-cap methyltransferase complex localization [GO:0070817] (biological process) Definition: Any process in which the P-TEFb-cap methyltransferase complex is transported to, or maintained in, a specific location. Sources: GOC:mah Also known as: P-TEFb-cap methyltransferase complex localisation, establishment and maintenance of P-TEFb-cap methyltransferase complex localization Relationships: is a type of GO:0031503